{
  "gene_name": "Apolipoprotein C-II",
  "term_label": "chylomicron",
  "term_id": "GO:0042627",
  "gene_symbol": "APOC2",
  "gene": "UniProtKB:P02655"
}